{
  "gene_name": "Olfactory receptor 4C11",
  "gene_symbol": "OR4C11",
  "gene": "UniProtKB:Q6IEV9",
  "term_label": "plasma membrane",
  "term_id": "GO:0005886"
}